{
  "gene_symbol": "CEP15",
  "gene": "UniProtKB:Q9HBI5",
  "gene_name": "Centrosomal protein 15 kDa",
  "term_id": "UNKNOWN:0002",
  "term_label": "Unknown biological process"
}